sno(s)RNA 3'-end processing [GO:0031126] (biological process) Relationships: is_a GO:0031123; is a type of sno(s)RNA processing [GO:0043144] Subtypes: box C/D sno(s)RNA 3'-end processing [GO:0000494], box H/ACA sno(s)RNA 3'-end processing [GO:0000495], sno(s)RNA 3'-end cleavage [GO:0043145], poly(A)-dependent snoRNA 3'-end processing [GO:0071051] References: PMID:17284456 Sources: GOC:krc, GOC:mah Definition: Any process involved in forming the mature 3' end of a snoRNA family molecule, also referred to as an sRNA in Archaea. Also known as: sno(s)RNA 3' end processing, sRNA 3'-end processing, snoRNA 3'-end processing